{
  "gene_name": "Troponin I, fast skeletal muscle",
  "gene": "UniProtKB:P48788",
  "term_id": "UNKNOWN:0001",
  "term_label": "Unknown molecular function",
  "gene_symbol": "TNNI2"
}